sieve plate [GO:0097218] (cellular component) Relationships: is a type of cellular anatomical structure [GO:0110165]; is part of GO:0009505; has part sieve area [GO:0097217] Subtypes: compound sieve plate [GO:0097219], simple sieve plate [GO:0097220] Note: Typical of angiosperms. Part of sieve tube member (PO:0000289). Definition: A part of the cell wall of a sieve tube member that bears one or more highly specialized sieve areas. Sources: ISBN:0471738433, POC:curators